{
  "term_label": "Unknown molecular function",
  "gene_name": "Transcription factor Gibbin",
  "gene_symbol": "AHDC1",
  "gene": "UniProtKB:Q5TGY3",
  "term_id": "UNKNOWN:0001"
}